{
  "gene": "UniProtKB:Q8WV60",
  "term_label": "regulation of mRNA processing",
  "gene_symbol": "PTCD2",
  "gene_name": "Pentatricopeptide repeat-containing protein 2, mitochondrial",
  "term_id": "GO:0050684"
}